guanosine-5'-triphosphate,3'-diphosphate diphosphatase activity [GO:0008894] (molecular function) Relationships: is_a GO:0016462 Sources: EC:3.6.1.40 Also known as: guanosine-5'-triphosphate,3'-diphosphate pyrophosphatase activity, guanosine 5'-triphosphate 3'-diphosphate 5'-phosphatase activity, guanosine 5'-triphosphate-3'-diphosphate 5'-phosphohydrolase activity, guanosine pentaphosphatase activity, guanosine pentaphosphate phosphatase activity, guanosine pentaphosphate phosphohydrolase activity, guanosine-5'-triphosphate,3'-diphosphate 5'-phosphohydrolase activity, pppGpp 5'-phosphohydrolase activity Definition: Catalysis of the reaction: guanosine 5'-triphosphate,3'-diphosphate + H2O = guanosine 5'-diphosphate,3'-diphosphate + phosphate.